{
  "gene": "UniProtKB:Q8IZ02",
  "gene_name": "Leucine-rich repeat-containing protein 34",
  "term_label": "Unknown biological process",
  "term_id": "UNKNOWN:0002",
  "gene_symbol": "LRRC34"
}